{
  "gene_name": "Fascin-2",
  "term_id": "GO:0007163",
  "term_label": "establishment or maintenance of cell polarity",
  "gene": "UniProtKB:O14926",
  "gene_symbol": "FSCN2"
}